{
  "term_label": "positive regulation of canonical Wnt signaling pathway",
  "gene_symbol": "GID8",
  "term_id": "GO:0090263",
  "gene_name": "Glucose-induced degradation protein 8 homolog",
  "gene": "UniProtKB:Q9NWU2"
}